kinesin II complex [GO:0016939] (cellular component) References: PMID:20930137 Definition: A complex consisting of two distinct motor subunits that form a heterodimer complexed with a third non-motor accessory subunit, the kinesin associated protein or KAP; the KIF3 heterodimer interacts via its C-terminal portion with KAP, which is thought to regulate the binding of the motor to cargo membranes. Relationships: is_a kinesin complex [GO:0005871]